{
  "term_id": "UNKNOWN:0002",
  "term_label": "Unknown biological process",
  "gene": "UniProtKB:Q9H813",
  "gene_symbol": "PACC1",
  "gene_name": "Proton-activated chloride channel"
}